{
  "term_id": "UNKNOWN:0003",
  "gene_name": "Zinc finger protein 138",
  "gene": "UniProtKB:P52744",
  "term_label": "Unknown cellular component",
  "gene_symbol": "ZNF138"
}